negative regulation of connective tissue replacement [GO:1905204] (BP) Also known as: down regulation of connective tissue replacement, down-regulation of connective tissue replacement, downregulation of connective tissue replacement, inhibition of connective tissue replacement References: PMID:25590961 Sources: GOC:BHF, GOC:BHF_miRNA, GOC:TermGenie, GOC:bc, GO_REF:0000058 Subtypes: GO:1904597 Definition: Any process that stops, prevents or reduces the frequency, rate or extent of connective tissue replacement. Relationships: is a type of negative regulation of tissue remodeling [GO:0034104]; is a type of regulation of connective tissue replacement [GO:1905203]; negatively regulates GO:0097709